{
  "gene_symbol": "COPA",
  "gene": "UniProtKB:P53621",
  "term_id": "GO:0006891",
  "term_label": "intra-Golgi vesicle-mediated transport",
  "gene_name": "Coatomer subunit alpha"
}